protein-DNA-RNA complex [GO:0001114] (cellular component) Sources: GOC:txnOH Definition: A macromolecular complex containing protein, DNA, and RNA molecules. Relationships: is a type of protein-containing complex [GO:0032991] Subtypes: transcription ternary complex [GO:0097523]